{
  "term_id": "GO:0005923",
  "gene_name": "Angiomotin-like protein 1",
  "gene": "UniProtKB:Q8IY63",
  "gene_symbol": "AMOTL1",
  "term_label": "bicellular tight junction"
}